arsenate reductase (azurin) activity [GO:0050611] (molecular function) Definition: Catalysis of the reaction: H2O + arsenite + 2 oxidized azurin = 2 H+ + 2 reduced azurin + arsenate. Sources: EC:1.20.9.1, MetaCyc:1.20.98.1-RXN Also known as: arsenite oxidase activity, arsenite:azurin oxidoreductase activity Relationships: is a type of oxidoreductase activity, acting on phosphorus or arsenic in donors, with a copper protein as acceptor [GO:0052882]